{
  "term_label": "Unknown molecular function",
  "gene_name": "WD repeat-containing protein 36",
  "gene_symbol": "WDR36",
  "gene": "UniProtKB:Q8NI36",
  "term_id": "UNKNOWN:0001"
}